{
  "gene_symbol": "ARHGAP35",
  "term_label": "GTPase activator activity",
  "term_id": "GO:0005096",
  "gene_name": "Rho GTPase-activating protein 35",
  "gene": "UniProtKB:Q9NRY4"
}